{
  "gene_symbol": "PPP1R9B",
  "gene_name": "Neurabin-2",
  "gene": "UniProtKB:Q96SB3",
  "term_id": "GO:0019722",
  "term_label": "calcium-mediated signaling"
}